type 2 metabotropic GABA receptor binding [GO:0031797] (molecular function) Definition: Binding to a type 2 metabotropic GABA receptor. Relationships: is a type of GO:0031795 Sources: GOC:mah, GOC:nln Also known as: type 2 metabotropic GABA receptor ligand